levan fructotransferase (DFA-IV-forming) activity [GO:0033996] (molecular function) Also known as: 2,6-beta-D-fructan D-fructosyl-D-fructosyltransferase (forming di-beta-D-fructofuranose 2,6':2',6-dianhydride) activity, 2,6-beta-D-fructan lyase (di-beta-D-fructofuranose-2,6':2',6-dianhydride-forming) activity, levan fructotransferase activity Definition: Catalysis of the reaction: beta-D-fructopyranosyl-(2->6)-[D-fructofuranosyl-(2->6)]n-D-fructofuranoside = beta-D-fructopyranosyl-(2->6)-[D-fructofuranosyl-(2->6)](n-1)-D-fructofuranoside + di-beta-D-fructofuranose 2,6':2',6-dianhydride. This reaction is the production of di-beta-D-fructofuranose 2,6':2',6-dianhydride (DFA IV) by successively eliminating the diminishing (2->6)-beta-D-fructan (levan) chain from the terminal D-fructosyl-D-fructosyl disaccharide. Sources: EC:4.2.2.16 Relationships: is a type of carbon-oxygen lyase activity, acting on polysaccharides [GO:0016837]